CoA-disulfide reductase (NADPH) activity [GO:0050451] (molecular function) Also known as: CoA-disulfide reductase activity, CoA-disulphide reductase activity, CoA-disulfide reductase (NADP) activity, CoA-disulfide reductase (NADH) activity, CoADR activity, NADH:CoA-disulfide oxidoreductase activity, coenzyme A disulfide reductase activity Definition: Catalysis of the reaction: 2 CoA + NADP+ = CoA-disulfide + NADPH + H+. Sources: RHEA:14705 Relationships: is a type of GO:0015036; is a type of oxidoreductase activity, acting on a sulfur group of donors, NAD(P) as acceptor [GO:0016668]